{
  "gene_name": "Signal peptide peptidase-like 2C",
  "term_id": "GO:0042500",
  "term_label": "aspartic endopeptidase activity, intramembrane cleaving",
  "gene_symbol": "SPPL2C",
  "gene": "UniProtKB:Q8IUH8"
}